negative regulation of telomerase catalytic core complex assembly [GO:1904883] (biological process) Also known as: down regulation of telomerase catalytic core complex assembly, down regulation of telomerase catalytic core complex formation, down-regulation of telomerase catalytic core complex assembly, down-regulation of telomerase catalytic core complex formation, downregulation of telomerase catalytic core complex assembly, downregulation of telomerase catalytic core complex formation, negative regulation of telomerase catalytic core complex formation, inhibition of telomerase catalytic core complex assembly, inhibition of telomerase catalytic core complex formation, down regulation of TERT-TERC complex assembly, down regulation of TERT-TERC complex formation, down-regulation of TERT-TERC complex assembly, down-regulation of TERT-TERC complex formation, downregulation of TERT-TERC complex assembly, downregulation of TERT-TERC complex formation, inhibition of TERT-TERC complex assembly, inhibition of TERT-TERC complex formation, negative regulation of TERT-TERC complex assembly, negative regulation of TERT-TERC complex formation Definition: Any process that stops, prevents or reduces the frequency, rate or extent of telomerase catalytic core complex assembly. Relationships: is a type of negative regulation of protein-containing complex assembly [GO:0031333]; is_a regulation of telomerase catalytic core complex assembly [GO:1904882]; negatively regulates telomerase catalytic core complex assembly [GO:1904868] References: PMID:26586433 Sources: GOC:BHF, GOC:BHF_telomere, GOC:TermGenie, GOC:rph, GO_REF:0000058